{
  "gene_symbol": "ABCG5",
  "gene_name": "ATP-binding cassette sub-family G member 5",
  "gene": "UniProtKB:Q9H222",
  "term_label": "ATPase-coupled transmembrane transporter activity",
  "term_id": "GO:0042626"
}